{
  "gene_name": "Lamin tail domain-containing protein 1",
  "gene_symbol": "LMNTD1",
  "term_id": "UNKNOWN:0001",
  "term_label": "Unknown molecular function",
  "gene": "UniProtKB:Q8N9Z9"
}